bacitracin A biosynthetic process [GO:1901124] (biological process) Relationships: is a type of amide biosynthetic process [GO:0043604] Sources: GOC:TermGenie, GOC:yaf, UniPathway:UPA00179 Definition: The chemical reactions and pathways resulting in the formation of bacitracin A. Also known as: bacitracin A anabolism, bacitracin A biosynthesis, bacitracin A formation, bacitracin A synthesis